tumor necrosis factor receptor superfamily binding [GO:0032813] (MF) Definition: Binding to a member of the tumor necrosis factor receptor superfamily. Sources: GOC:add Also known as: TNF receptor superfamily binding Subtypes: GO:0005123, tumor necrosis factor receptor binding [GO:0005164], CD40 receptor binding [GO:0005174], GO:0005175 Relationships: is a type of GO:0005126